{
  "gene_name": "3-hydroxyanthranilate 3,4-dioxygenase",
  "term_id": "GO:0000334",
  "gene": "UniProtKB:P46952",
  "gene_symbol": "HAAO",
  "term_label": "3-hydroxyanthranilate 3,4-dioxygenase activity"
}